{
  "term_id": "UNKNOWN:0002",
  "gene_symbol": "ANGPTL7",
  "term_label": "Unknown biological process",
  "gene": "UniProtKB:O43827",
  "gene_name": "Angiopoietin-related protein 7"
}